selenocysteine insertion sequence binding [GO:0035368] (molecular function) References: PMID:10760958 Sources: GOC:imk Relationships: is a type of mRNA binding [GO:0003729] Definition: Binding to a selenocysteine insertion sequence (SECIS), a regulatory sequence within mRNA which directs incorporation of a selenocysteine at a stop codon (UGA) during translation. Also known as: SECIS binding